peptidyl-threonine O-acetylation [GO:0120258] (biological process) Definition: The acetylation of peptidyl-threonine to form peptidyl-O-acetyl-L-threonine. Relationships: is a type of peptidyl-threonine modification [GO:0018210]; is a type of peptidyl-threonine acetylation [GO:0120257] References: PMID:16728640, PMID:22802624 Sources: RESID:AA0423